{
  "gene_symbol": "SIX6OS1",
  "term_id": "GO:0010705",
  "gene_name": "Protein SIX6OS1",
  "gene": "UniProtKB:Q8N1H7",
  "term_label": "meiotic DNA double-strand break processing involved in reciprocal meiotic recombination"
}